{
  "gene_name": "TATA box-binding protein-associated factor RNA polymerase I subunit B",
  "gene_symbol": "TAF1B",
  "term_label": "RNA polymerase I core factor complex",
  "gene": "UniProtKB:Q53T94",
  "term_id": "GO:0070860"
}